{
  "term_id": "GO:0016491",
  "term_label": "oxidoreductase activity",
  "gene_symbol": "CYB561D1",
  "gene_name": "Probable transmembrane reductase CYB561D1",
  "gene": "UniProtKB:Q8N8Q1"
}